{
  "gene": "UniProtKB:Q09472",
  "term_label": "positive regulation of transcription by RNA polymerase II",
  "gene_name": "Histone acetyltransferase p300",
  "term_id": "GO:0045944",
  "gene_symbol": "EP300"
}